{
  "gene": "UniProtKB:O43823",
  "term_id": "GO:0007076",
  "gene_symbol": "AKAP8",
  "gene_name": "A-kinase anchor protein 8",
  "term_label": "mitotic chromosome condensation"
}